histone dopaminyltransferase activity [GO:0120297] (MF) Relationships: is a type of peptide dopaminyltransferase activity [GO:0120296]; is a type of GO:0140993 References: PMID:32273471 Sources: GOC:sp Definition: Catalysis of the reaction: dopamine + L-glutaminyl-[histone] = 5-dopaminyl-L-glutamyl-[histone] + NH4(+).